{
  "gene_name": "Protein FAM193B",
  "gene": "UniProtKB:Q96PV7",
  "term_id": "UNKNOWN:0002",
  "term_label": "Unknown biological process",
  "gene_symbol": "FAM193B"
}